{
  "term_label": "phosphotransferase activity, for other substituted phosphate groups",
  "gene_name": "Ribitol 5-phosphate transferase FKRP",
  "term_id": "GO:0016780",
  "gene": "UniProtKB:Q9H9S5",
  "gene_symbol": "FKRP"
}